{
  "gene_symbol": "ZNF449",
  "gene": "UniProtKB:Q6P9G9",
  "gene_name": "Zinc finger protein 449",
  "term_label": "regulation of transcription by RNA polymerase II",
  "term_id": "GO:0006357"
}